{
  "gene": "UniProtKB:Q9UDX4",
  "gene_name": "SEC14-like protein 3",
  "gene_symbol": "SEC14L3",
  "term_label": "Unknown biological process",
  "term_id": "UNKNOWN:0002"
}